{
  "gene_name": "T cell receptor delta constant",
  "gene": "UniProtKB:B7Z8K6",
  "term_label": "Unknown molecular function",
  "term_id": "UNKNOWN:0001",
  "gene_symbol": "TRDC"
}